prostaglandin D receptor activity [GO:0004956] (molecular function) Definition: Combining with prostaglandin D (PGD(2)) to initiate a change in cell activity. Sources: ISBN:0198506732 Also known as: PGD(2) receptor activity, PGD receptor activity Relationships: is a type of prostaglandin receptor activity [GO:0004955]